{
  "term_label": "TIM23 mitochondrial import inner membrane translocase complex",
  "gene_name": "Reactive oxygen species modulator 1",
  "gene": "UniProtKB:P60602",
  "gene_symbol": "ROMO1",
  "term_id": "GO:0005744"
}